{
  "term_id": "GO:0005634",
  "gene_symbol": "ZNF493",
  "gene_name": "Zinc finger protein 493",
  "gene": "UniProtKB:Q6ZR52",
  "term_label": "nucleus"
}